{
  "gene": "UniProtKB:Q9UJW0",
  "term_id": "GO:0005869",
  "gene_symbol": "DCTN4",
  "term_label": "dynactin complex",
  "gene_name": "Dynactin subunit 4"
}